{
  "term_id": "GO:0008253",
  "gene_symbol": "NT5DC2",
  "gene_name": "5'-nucleotidase domain-containing protein 2",
  "gene": "UniProtKB:Q9H857",
  "term_label": "5'-nucleotidase activity"
}